{
  "gene": "UniProtKB:Q9NQ11",
  "gene_name": "Polyamine-transporting ATPase 13A2",
  "term_label": "ATPase-coupled monoatomic cation transmembrane transporter activity",
  "gene_symbol": "ATP13A2",
  "term_id": "GO:0019829"
}